{
  "term_id": "UNKNOWN:0003",
  "term_label": "Unknown cellular component",
  "gene_name": "AP-4 complex subunit beta-1",
  "gene_symbol": "AP4B1",
  "gene": "UniProtKB:Q9Y6B7"
}